{
  "gene_symbol": "CYP2D7",
  "term_id": "GO:0016712",
  "gene_name": "Putative cytochrome P450 2D7",
  "gene": "UniProtKB:A0A087X1C5",
  "term_label": "oxidoreductase activity, acting on paired donors, with incorporation or reduction of molecular oxygen, reduced flavin or flavoprotein as one donor, and incorporation of one atom of oxygen"
}